symbiont-mediated perturbation of host immune response [GO:0052553] (biological process) Also known as: modulation by organism of immune response of other organism involved in symbiotic interaction, modulation by symbiont of host immune response, perturbation of host immune response Subtypes: symbiont-mediated evasion of host immune response [GO:0042783], symbiont-mediated perturbation of host B-cell mediated immune response [GO:0052154], symbiont-mediated perturbation of host T-cell mediated immune response [GO:0052156], symbiont-mediated perturbation of host induced systemic resistance [GO:0052159], symbiont-mediated perturbation of host innate immune response [GO:0052167], symbiont-mediated suppression of host immune response [GO:0052562], symbiont-mediated non-specific activation of host T-cells [GO:0141128] Relationships: is_a symbiont-mediated perturbation of host defense response [GO:0052031] Definition: A process in which a symbiont alters or subverts the immune response of the host organism; the immune response is any immune system process that functions in the calibrated response of an organism to a potential internal or invasive threat. The host is defined as the larger of the organisms involved in a symbiotic interaction. Sources: GOC:mtg_pamgo_17jul06